{
  "term_id": "GO:0005789",
  "gene_name": "cTAGE family member 9",
  "gene": "UniProtKB:A4FU28",
  "term_label": "endoplasmic reticulum membrane",
  "gene_symbol": "CTAGE9"
}